{
  "term_id": "GO:0050804",
  "term_label": "modulation of chemical synaptic transmission",
  "gene": "UniProtKB:Q8TCU5",
  "gene_name": "Glutamate receptor ionotropic, NMDA 3A",
  "gene_symbol": "GRIN3A"
}